mitochondrial large ribosomal subunit assembly [GO:1902775] (biological process) Definition: The aggregation, arrangement and bonding together of a set of components to form a mitochondrial large ribosomal subunit. References: PMID:24206665 Sources: GOC:TermGenie, GO_REF:0000079 Relationships: is a type of ribosomal large subunit assembly [GO:0000027]; is part of mitochondrial ribosome assembly [GO:0061668] Also known as: mitochondrial large ribosomal subunit formation, 39S ribosomal subunit, mitochondrial assembly, 39S ribosomal subunit, mitochondrial formation